{
  "gene_name": "Putative dispanin subfamily A member 2d",
  "term_id": "GO:0051607",
  "gene_symbol": "C9JQL5",
  "term_label": "defense response to virus",
  "gene": "UniProtKB:C9JQL5"
}